protein-lipid complex binding [GO:0071814] (molecular function) Sources: GOC:BHF, GOC:mah Relationships: is a type of protein-containing complex binding [GO:0044877] Definition: Binding to a protein-lipid complex, any macromolecular complex that contains both protein and lipid molecules. Subtypes: lipoprotein particle binding [GO:0071813]